glutamate metabolic process [GO:0006536] (biological process) Regulation: regulated by regulation of glutamate metabolic process [GO:2000211]; RO_0002212 by negative regulation of glutamate metabolic process [GO:2000212] Sources: GOC:go_curators Definition: The chemical reactions and pathways involving glutamate, the anion of 2-aminopentanedioic acid. Relationships: is a type of glutamine family amino acid metabolic process [GO:0009064]; is a type of dicarboxylic acid metabolic process [GO:0043648] Also known as: glutamate metabolism, glutamic acid metabolic process, glutamic acid metabolism Subtypes: glutamate biosynthetic process [GO:0006537], L-glutamate catabolic process [GO:0006538], GO:0010133, GO:0019544, glutamate catabolic process to oxaloacetate [GO:0019554], L-histidine catabolic process to glutamate and formamide [GO:0019556], L-histidine catabolic process to glutamate and formate [GO:0019557], GO:0019676, GO:0033526